{
  "term_label": "nucleus",
  "term_id": "GO:0005634",
  "gene": "UniProtKB:Q9NTG7",
  "gene_name": "NAD-dependent protein deacetylase sirtuin-3, mitochondrial",
  "gene_symbol": "SIRT3"
}